{
  "gene_symbol": "ANXA2P2",
  "gene": "UniProtKB:A6NMY6",
  "gene_name": "Putative annexin A2-like protein",
  "term_label": "phosphatidylserine binding",
  "term_id": "GO:0001786"
}